{
  "gene_name": "Tetraspanin-31",
  "gene_symbol": "TSPAN31",
  "term_id": "UNKNOWN:0002",
  "term_label": "Unknown biological process",
  "gene": "UniProtKB:Q12999"
}